succinate-CoA ligase complex [GO:0042709] (cellular component) Relationships: is a type of tricarboxylic acid cycle heteromeric enzyme complex [GO:0045239] Definition: A heterodimeric enzyme complex, usually composed of an alpha and beta chain. Functions in the TCA cycle, hydrolyzing succinyl-CoA into succinate and CoA, thereby forming ATP or GTP. Subtypes: succinate-CoA ligase complex (ADP-forming) [GO:0009361], succinate-CoA ligase complex (GDP-forming) [GO:0045244] References: PMID:10671455 Sources: GOC:jl